{
  "gene_name": "Secretion-regulating guanine nucleotide exchange factor",
  "term_id": "GO:0050709",
  "term_label": "negative regulation of protein secretion",
  "gene": "UniProtKB:Q9UGK8",
  "gene_symbol": "SERGEF"
}